{
  "gene_symbol": "CAPN5",
  "gene": "UniProtKB:O15484",
  "term_id": "GO:0006508",
  "term_label": "proteolysis",
  "gene_name": "Calpain-5"
}